{
  "term_id": "GO:0045505",
  "term_label": "dynein intermediate chain binding",
  "gene_symbol": "DYNLT3",
  "gene_name": "Dynein light chain Tctex-type 3",
  "gene": "UniProtKB:P51808"
}